{
  "gene": "UniProtKB:A0A286YF77",
  "gene_name": "Small cysteine and glycine repeat-containing protein 6",
  "term_id": "UNKNOWN:0001",
  "term_label": "Unknown molecular function",
  "gene_symbol": "SCYGR6"
}